fast, calcium ion-dependent exocytosis of neurotransmitter [GO:0098746] (biological process) Definition: The fast, initial phase of calcium ion-induced neurotransmitter release, via exocytosis, into the synaptic cleft. This depends on low affinity calcium sensors and typically begins a fraction of a millisecond after Ca2+ influx, and decays rapidly (1-10ms) with a decay constant of around 5-10ms. The underlying molecular mechanisms of this process are distinct from those of the later, slow phase of release. References: PMID:4405553, PMID:7809151, PMID:7954835 Sources: GOC:PARL, GOC:dos, GOC:pad Also known as: synchronous, calcium ion-dependent exocytosis of neurotransmitter Relationships: is a type of calcium ion-regulated exocytosis of neurotransmitter [GO:0048791]